{
  "gene_symbol": "MARS2",
  "term_id": "GO:0006431",
  "gene_name": "Methionine--tRNA ligase, mitochondrial",
  "gene": "UniProtKB:Q96GW9",
  "term_label": "methionyl-tRNA aminoacylation"
}